positive regulation of DNA strand elongation [GO:0060383] (biological process) Sources: GOC:mah Definition: Any process that increases the rate, frequency or extent of DNA strand elongation. DNA strand elongation is the DNA metabolic process in which an existing DNA strand is extended by activities including the addition of nucleotides to the 3' end of the strand. Relationships: is a type of positive regulation of DNA metabolic process [GO:0051054]; is a type of GO:0060382; positively regulates DNA strand elongation [GO:0022616]